{
  "term_label": "proteasome regulatory particle, base subcomplex",
  "gene_name": "26S proteasome non-ATPase regulatory subunit 1",
  "gene": "UniProtKB:Q99460",
  "gene_symbol": "PSMD1",
  "term_id": "GO:0008540"
}